{
  "gene": "UniProtKB:Q8IZF2",
  "gene_name": "Adhesion G protein-coupled receptor F5",
  "term_label": "surfactant homeostasis",
  "gene_symbol": "ADGRF5",
  "term_id": "GO:0043129"
}